symbiont-mediated migration across host tissue barrier [GO:0141142] (biological process) Subtypes: GO:0035756 Definition: A process in which a symbiont moves across a tissue barrier of the host to transports itself across an extracellular cellular matrix barrier or between the cells of a tissue. This involves the temporary or permanent breaching of the tissue barrier. Relationships: is a type of migration in host [GO:0044001] References: PMID:19820089, PMID:20188700, PMID:26681776, PMID:29120408